ciliary vesicle assembly [GO:1905556] (biological process) Definition: The aggregation, arrangement and bonding together of a set of components to form a ciliary vesicle. Multiple smaller vesicles dock to the transitional fibers on a mature basal body and then fuse together to form a larger single vesicle. This then fuses with the plasma membrane and forms the ciliary membrane. References: PMID:13978319, PMID:25313408, PMID:25805133, PMID:25812525 Sources: GOC:TermGenie, GOC:cilia, GO_REF:0000079 Also known as: ciliary vesicle formation, primary ciliary vesicle assembly, primary ciliary vesicle formation, CV assembly, CV formation Relationships: is_a vesicle organization [GO:0016050]; is a type of organelle assembly [GO:0070925]